nuclear chromosome segregation [GO:0098813] (biological process) Definition: The process in which genetic material, in the form of nuclear chromosomes, is organized into specific structures and then physically separated and apportioned to two or more sets. Nuclear chromosome segregation begins with the condensation of chromosomes, includes chromosome separation, and ends when chromosomes have completed movement to the spindle poles. Subtypes: sister chromatid segregation [GO:0000819], meiotic chromosome segregation [GO:0045132] Relationships: is a type of chromosome segregation [GO:0007059] Sources: GOC:dos